{
  "gene": "UniProtKB:Q15392",
  "term_label": "Delta24(24-1) sterol reductase activity",
  "gene_symbol": "DHCR24",
  "gene_name": "Delta(24)-sterol reductase",
  "term_id": "GO:0000246"
}